aspartic acid methylthiotransferase activity [GO:0035599] (molecular function) Definition: Catalysis of the methylthiolation (-SCH3 addition) of the beta-carbon of peptidyl-aspartic acid to form peptidyl-L-beta-methylthioaspartic acid. References: PMID:18252828, PMID:8844851 Sources: RESID:AA0232 Note: Note that peptidyl-L-beta-methylthioaspartic acid is typical of bacterial ribosomal protein S12. Relationships: is_a methylthiotransferase activity [GO:0035596]; is part of peptidyl-L-beta-methylthioaspartic acid biosynthetic process from peptidyl-aspartic acid [GO:0018339]